{
  "gene": "UniProtKB:Q8IYE1",
  "term_id": "GO:1905515",
  "gene_name": "Coiled-coil domain-containing protein 13",
  "gene_symbol": "CCDC13",
  "term_label": "non-motile cilium assembly"
}